{
  "gene_name": "Purine-rich element-binding protein gamma",
  "term_id": "GO:0000977",
  "gene": "UniProtKB:Q9UJV8",
  "term_label": "RNA polymerase II transcription regulatory region sequence-specific DNA binding",
  "gene_symbol": "PURG"
}